{
  "gene": "UniProtKB:Q9NSD5",
  "gene_symbol": "SLC6A13",
  "gene_name": "Sodium- and chloride-dependent GABA transporter 2",
  "term_id": "GO:0042995",
  "term_label": "cell projection"
}